{
  "gene_name": "Intersectin-2",
  "term_id": "GO:0097708",
  "term_label": "intracellular vesicle",
  "gene_symbol": "ITSN2",
  "gene": "UniProtKB:Q9NZM3"
}